{
  "term_id": "GO:0003924",
  "term_label": "GTPase activity",
  "gene": "UniProtKB:P08754",
  "gene_name": "Guanine nucleotide-binding protein G(i) subunit alpha-3",
  "gene_symbol": "GNAI3"
}